glial cell apoptotic process [GO:0034349] (biological process) Sources: CL:0000125, GOC:mtg_apoptosis, GOC:sart Also known as: apoptosis of glia, apoptosis of glial cells, glia apoptosis, glia programmed cell death by apoptosis, glial cell programmed cell death by apoptosis, programmed cell death of glia by apoptosis, programmed cell death of glial cells by apoptosis, programmed cell death, glia, programmed cell death, glial cells, glial cell apoptosis Relationships: is a type of GO:0006915 Regulation: regulated by GO:0034350; negatively regulated by negative regulation of glial cell apoptotic process [GO:0034351]; positively regulated by GO:0034352 Subtypes: oligodendrocyte apoptotic process [GO:0097252] Definition: Any apoptotic process in a glial cell, a non-neuronal cell of the nervous system.